{
  "gene": "UniProtKB:O95251",
  "term_id": "GO:0010484",
  "gene_name": "Histone acetyltransferase KAT7",
  "term_label": "histone H3 acetyltransferase activity",
  "gene_symbol": "KAT7"
}